{
  "term_id": "GO:0005814",
  "term_label": "centriole",
  "gene_name": "Centriole, cilia and spindle-associated protein",
  "gene": "UniProtKB:Q6IQ19",
  "gene_symbol": "CCSAP"
}